{
  "gene_symbol": "ADM",
  "term_id": "GO:0005615",
  "gene": "UniProtKB:P35318",
  "term_label": "extracellular space",
  "gene_name": "Pro-adrenomedullin"
}